regulation of T-helper 1 cell activation [GO:2000517] (biological process) Sources: GOC:obol Relationships: is a type of regulation of CD4-positive, alpha-beta T cell activation [GO:2000514]; RO_0002211 T-helper 1 cell activation [GO:0035711] Definition: Any process that modulates the frequency, rate or extent of T-helper 1 cell activation. Subtypes: GO:2000518, GO:2000519 Also known as: regulation of Th1 cell activation